{
  "gene_symbol": "SMARCB1",
  "gene": "UniProtKB:Q12824",
  "term_id": "GO:0071564",
  "term_label": "npBAF complex",
  "gene_name": "SWI_SNF-related matrix-associated actin-dependent regulator of chromatin subfamily B member 1"
}